{
  "gene_symbol": "MGAT4B",
  "term_label": "endoplasmic reticulum",
  "gene_name": "Alpha-1,3-mannosyl-glycoprotein 4-beta-N-acetylglucosaminyltransferase B",
  "term_id": "GO:0005783",
  "gene": "UniProtKB:Q9UQ53"
}